{
  "gene_name": "CCN family member 5",
  "term_id": "GO:0045597",
  "gene_symbol": "CCN5",
  "gene": "UniProtKB:O76076",
  "term_label": "positive regulation of cell differentiation"
}